{
  "term_id": "UNKNOWN:0001",
  "gene_name": "Disabled homolog 1",
  "gene": "UniProtKB:O75553",
  "gene_symbol": "DAB1",
  "term_label": "Unknown molecular function"
}